{
  "term_label": "Golgi to plasma membrane transport",
  "gene_symbol": "CCDC93",
  "term_id": "GO:0006893",
  "gene": "UniProtKB:Q567U6",
  "gene_name": "Coiled-coil domain-containing protein 93"
}